{
  "gene_name": "X-linked retinitis pigmentosa GTPase regulator",
  "term_label": "visual perception",
  "term_id": "GO:0007601",
  "gene": "UniProtKB:Q92834",
  "gene_symbol": "RPGR"
}